regulation of inflorescence meristem growth [GO:0010081] (biological process) Relationships: is a type of regulation of meristem growth [GO:0010075]; is_a regulation of reproductive process [GO:2000241]; regulates GO:0010450 Also known as: regulation of inflorescence meristem size Sources: GOC:tb Definition: Any process involved in maintaining the size and shape of an inflorescence meristem.